{
  "term_id": "UNKNOWN:0002",
  "term_label": "Unknown biological process",
  "gene": "UniProtKB:Q96D70",
  "gene_symbol": "R3HDM4",
  "gene_name": "R3H domain-containing protein 4"
}